procollagen glucosyltransferase activity [GO:0033823] (molecular function) Sources: EC:2.4.1.66 Definition: Catalysis of the reaction: UDP-glucose + 5-(D-galactosyloxy)-L-lysine-procollagen = UDP + 1,2-D-glucosyl-5-D-(galactosyloxy)-L-lysine-procollagen. Also known as: UDP-glucose-collagenglucosyltransferase activity, UDP-glucose:5-(D-galactosyloxy)-L-lysine-procollagen D-glucosyltransferase activity, UDPglucose:5-(D-galactosyloxy)-L-lysine-procollagen D-glucosyltransferase activity, collagen glucosyltransferase activity, collagen hydroxylysyl glucosyltransferase activity, galactosylhydroxylysine glucosyltransferase activity, galactosylhydroxylysine-glucosyltransferase activity, galactosylhydroxylysyl glucosyltransferase activity, uridine diphosphoglucose-collagen glucosyltransferase activity Relationships: is a type of GO:0046527; is a type of GO:0140096